{
  "term_label": "cyclin E1-CDK2 complex",
  "term_id": "GO:0097134",
  "gene_symbol": "CCNE1",
  "gene": "UniProtKB:P24864",
  "gene_name": "G1_S-specific cyclin-E1"
}